{
  "term_label": "oxidoreductase activity, acting on the CH-OH group of donors, NAD or NADP as acceptor",
  "gene": "UniProtKB:Q8N4T8",
  "gene_name": "3-oxoacyl-[acyl-carrier-protein] reductase",
  "term_id": "GO:0016616",
  "gene_symbol": "CBR4"
}